{
  "gene_symbol": "TEX11",
  "gene": "UniProtKB:Q8IYF3",
  "gene_name": "Testis-expressed protein 11",
  "term_label": "Unknown molecular function",
  "term_id": "UNKNOWN:0001"
}